{
  "gene_symbol": "OXTR",
  "term_label": "G protein-coupled receptor signaling pathway",
  "gene": "UniProtKB:P30559",
  "gene_name": "Oxytocin receptor",
  "term_id": "GO:0007186"
}